{
  "term_label": "spermatogenesis",
  "term_id": "GO:0007283",
  "gene_symbol": "TDRD1",
  "gene": "UniProtKB:Q9BXT4",
  "gene_name": "Tudor domain-containing protein 1"
}